{
  "term_id": "GO:0016320",
  "gene": "UniProtKB:Q96JH7",
  "gene_name": "Deubiquitinating protein VCPIP1",
  "gene_symbol": "VCPIP1",
  "term_label": "endoplasmic reticulum membrane fusion"
}